{
  "gene_symbol": "SEMA3E",
  "term_label": "neuropilin binding",
  "gene": "UniProtKB:O15041",
  "gene_name": "Semaphorin-3E",
  "term_id": "GO:0038191"
}